{
  "gene_symbol": "SLC24A3",
  "gene": "UniProtKB:Q9HC58",
  "term_id": "GO:0008273",
  "gene_name": "Sodium_potassium_calcium exchanger 3",
  "term_label": "calcium, potassium:sodium antiporter activity"
}